{
  "gene": "UniProtKB:Q6P6C2",
  "term_label": "oxidative RNA demethylase activity",
  "gene_name": "RNA demethylase ALKBH5",
  "term_id": "GO:0035515",
  "gene_symbol": "ALKBH5"
}